{
  "term_id": "UNKNOWN:0002",
  "gene_symbol": "SNX19",
  "gene": "UniProtKB:Q92543",
  "gene_name": "Sorting nexin-19",
  "term_label": "Unknown biological process"
}